{
  "gene": "UniProtKB:A0A0K0K1G8",
  "term_id": "GO:0005886",
  "gene_name": "T cell receptor beta variable 10-2",
  "gene_symbol": "TRBV10-2",
  "term_label": "plasma membrane"
}